{
  "gene_symbol": "CNTN2",
  "term_id": "GO:0007411",
  "gene_name": "Contactin-2",
  "term_label": "axon guidance",
  "gene": "UniProtKB:Q02246"
}